cellular response to methotrexate [GO:0071414] (biological process) Relationships: is a type of response to methotrexate [GO:0031427]; is a type of GO:1901699; is a type of cellular response to oxygen-containing compound [GO:1901701] Definition: Any process that results in a change in state or activity of a cell (in terms of movement, secretion, enzyme production, gene expression, etc.) as a result of a methotrexate stimulus. Methotrexate is 4-amino-10-methylformic acid, a folic acid analogue that is a potent competitive inhibitor of dihydrofolate reductase. Sources: GOC:mah